formyltetrahydrofolate deformylase activity [GO:0008864] (molecular function) Definition: Catalysis of the reaction: 10-formyltetrahydrofolate + H2O = (6S)-5,6,7,8-tetrahydrofolate + formate + H+. Also known as: 10-formyltetrahydrofolate amidohydrolase activity, formyl-FH(4) hydrolase activity, formyltetrahydrofolate hydrolase activity Relationships: is a type of hydrolase activity, acting on carbon-nitrogen (but not peptide) bonds, in linear amides [GO:0016811] Sources: EC:3.5.1.10, RHEA:19833